type 1B melatonin receptor binding [GO:0031786] (molecular function) Sources: GOC:mah, GOC:nln Relationships: is a type of melatonin receptor binding [GO:0031784] Also known as: type 1B melatonin receptor ligand Definition: Binding to a type 1B melatonin receptor.